negative regulation of vein smooth muscle contraction [GO:0062088] (biological process) Relationships: is a type of regulation of vein smooth muscle contraction [GO:0062086]; is a type of negative regulation of vascular associated smooth muscle contraction [GO:1904694]; negatively regulates GO:0014826 References: PMID:8428203 Definition: Any process that decreases the frequency, rate or extent of vein smooth muscle contraction.